CCC codon-amino acid adaptor activity [GO:0033422] (molecular function) Sources: GOC:mah Definition: A triplet codon-amino acid adaptor activity that recognizes a CCC codon. Also known as: proline tRNA Relationships: is a type of GO:0030533 Note: Note that in the standard genetic code, CCC codes for proline.